{
  "term_id": "GO:1990756",
  "term_label": "ubiquitin-like ligase-substrate adaptor activity",
  "gene_name": "Kelch-like protein 8",
  "gene": "UniProtKB:Q9P2G9",
  "gene_symbol": "KLHL8"
}